{
  "term_id": "GO:0043161",
  "gene": "UniProtKB:Q9Y573",
  "term_label": "proteasome-mediated ubiquitin-dependent protein catabolic process",
  "gene_symbol": "IPP",
  "gene_name": "Actin-binding protein IPP"
}